L-rhamnono-1,4-lactonase activity [GO:0050033] (molecular function) Sources: EC:3.1.1.65, RHEA:10288 Relationships: is a type of carboxylic ester hydrolase activity [GO:0052689] Also known as: L-rhamno-gamma-lactonase activity, L-rhamnono-1,4-lactone lactonohydrolase activity, L-rhamnono-gamma-lactonase activity Definition: Catalysis of the reaction: L-rhamnono-1,4-lactone + H2O = L-rhamnonate + H+.